{
  "gene": "UniProtKB:Q9BQ13",
  "term_id": "UNKNOWN:0003",
  "gene_name": "BTB_POZ domain-containing protein KCTD14",
  "term_label": "Unknown cellular component",
  "gene_symbol": "KCTD14"
}